protection from non-homologous end joining at telomere [GO:0031848] (biological process) Sources: GOC:mah Definition: A process that prevents non-homologous end joining at telomere, thereby ensuring that telomeres do not fuse. Also known as: protection from NHEJ-mediated telomere fusion Relationships: is a type of telomere maintenance in response to DNA damage [GO:0043247]; is part of telomere capping [GO:0016233] Regulation: regulated by regulation of protection from non-homologous end joining at telomere [GO:1905764]; negatively regulated by GO:1905765; RO_0002213 by positive regulation of protection from non-homologous end joining at telomere [GO:1905766]